{
  "term_label": "Unknown cellular component",
  "term_id": "UNKNOWN:0003",
  "gene_symbol": "TRAJ13",
  "gene_name": "T cell receptor alpha joining 13 (Fragment)",
  "gene": "UniProtKB:A0A075B709"
}